{
  "term_label": "ubiquitin protein ligase activity",
  "term_id": "GO:0061630",
  "gene_symbol": "HUWE1",
  "gene_name": "E3 ubiquitin-protein ligase HUWE1",
  "gene": "UniProtKB:Q7Z6Z7"
}